{
  "term_label": "defense response to bacterium",
  "term_id": "GO:0042742",
  "gene": "UniProtKB:Q8TAX9",
  "gene_name": "Gasdermin-B",
  "gene_symbol": "GSDMB"
}